{
  "term_id": "GO:0003924",
  "gene": "UniProtKB:A6NIZ1",
  "term_label": "GTPase activity",
  "gene_name": "Ras-related protein Rap-1b-like protein",
  "gene_symbol": "RAP1BL"
}